symbiont-mediated suppression of host tumor necrosis factor-mediated signaling pathway [GO:0141072] (biological process) Definition: A process in which a virus interferes with, inhibits or disrupts a tumor necrosis factor-mediated signal transduction in its host organism. The host is defined as the larger of the organisms involved in a symbiotic interaction. Relationships: is a type of GO:0052029 References: PMID:11805081, PMID:24736233 Also known as: disruption of host TNF-mediated signaling pathway, disruption of host TNFR-mediated signaling pathway, disruption of host tumor necrosis factor receptor-mediated signaling pathway, disruption of host tumor necrosis factor-mediated signaling pathway